{
  "term_id": "GO:0034236",
  "gene_name": "cAMP-dependent protein kinase type I-beta regulatory subunit",
  "gene_symbol": "PRKAR1B",
  "gene": "UniProtKB:P31321",
  "term_label": "protein kinase A catalytic subunit binding"
}